type I hypersensitivity mediated by basophils [GO:0002559] (biological process) Sources: GOC:add, ISBN:0781735149 Relationships: is a type of basophil mediated immunity [GO:0002560]; is a type of type I hypersensitivity [GO:0016068] Definition: An inflammatory response driven by antigen recognition by antibodies bound to Fc receptors basophils, occurring within minutes after exposure of a sensitized individual to the antigen, and leading to the release of a variety of inflammatory mediators such as histamines.